{
  "term_id": "GO:0030027",
  "gene": "UniProtKB:Q6F5E8",
  "gene_symbol": "CARMIL2",
  "gene_name": "Capping protein, Arp2_3 and myosin-I linker protein 2",
  "term_label": "lamellipodium"
}